regulation of intracellular cholesterol transport [GO:0032383] (biological process) Subtypes: negative regulation of intracellular cholesterol transport [GO:0032384], GO:0032385 Relationships: is a type of regulation of cholesterol transport [GO:0032374]; is a type of regulation of intracellular sterol transport [GO:0032380]; regulates intracellular cholesterol transport [GO:0032367] Sources: GOC:mah Definition: Any process that modulates the frequency, rate or extent of the directed movement of cholesterol within cells.